{
  "term_id": "GO:0005886",
  "gene_symbol": "HTR5A",
  "term_label": "plasma membrane",
  "gene_name": "5-hydroxytryptamine receptor 5A",
  "gene": "UniProtKB:P47898"
}